negative regulation of amine transport [GO:0051953] (biological process) Relationships: is a type of negative regulation of transport [GO:0051051]; is a type of GO:0051952; RO_0002212 amine transport [GO:0015837] Definition: Any process that stops, prevents, or reduces the frequency, rate or extent of the directed movement of amines into, out of or within a cell, or between cells, by means of some agent such as a transporter or pore. Sources: GOC:ai Subtypes: negative regulation of acetylcholine secretion, neurotransmission [GO:0014058], negative regulation of catecholamine secretion [GO:0033604], negative regulation of acetylcholine uptake [GO:0051632], negative regulation of catecholamine uptake involved in synaptic transmission [GO:0051945], negative regulation of amino acid transport [GO:0051956] Also known as: down regulation of amine transport, down-regulation of amine transport, downregulation of amine transport, inhibition of amine transport